{
  "gene": "UniProtKB:P31513",
  "gene_name": "Flavin-containing monooxygenase 3",
  "gene_symbol": "FMO3",
  "term_id": "UNKNOWN:0003",
  "term_label": "Unknown cellular component"
}